{
  "gene_name": "Fc receptor-like protein 1",
  "term_label": "immune response",
  "term_id": "GO:0006955",
  "gene": "UniProtKB:Q96LA6",
  "gene_symbol": "FCRL1"
}